sodium:proton antiporter activity [GO:0015385] (molecular function) Definition: Enables the transfer of a solute or solutes from one side of a membrane to the other according to the reaction: Na+(out) + H+(in) = Na+(in) + H+(out). Relationships: is a type of sodium ion transmembrane transporter activity [GO:0015081]; is_a GO:0051139 Subtypes: sodium:proton antiporter activity involved in regulation of cardiac muscle cell membrane potential [GO:0086040], GO:0140830, GO:0140831, L-histidine, sodium:proton antiporter activity [GO:0140832], neutral amino acid, sodium:proton antiporter activity [GO:0140893] Regulation: positively regulated by positive regulation of sodium:proton antiporter activity [GO:0032417] Sources: TC:2.A.35.1.1, TC:2.A.36.-.- Also known as: sodium/hydrogen antiporter activity, sodium:hydrogen antiporter activity, sodium:hydrogen exchange activity, sodium:hydrogen exchanger, pH-dependent sodium:hydrogen antiporter activity, pH-dependent sodium:proton antiporter activity